{
  "term_id": "GO:0035925",
  "term_label": "mRNA 3'-UTR AU-rich region binding",
  "gene": "UniProtKB:Q96B26",
  "gene_symbol": "EXOSC8",
  "gene_name": "Exosome complex component RRP43"
}